{
  "term_id": "UNKNOWN:0001",
  "gene_symbol": "VMO1",
  "gene": "UniProtKB:Q7Z5L0",
  "gene_name": "Vitelline membrane outer layer protein 1 homolog",
  "term_label": "Unknown molecular function"
}